somatic recombination of immunoglobulin gene segments [GO:0016447] (biological process) Definition: The process in which immunoglobulin genes are formed through recombination of the germline genetic elements, as known as immunoglobulin gene segments, within a single locus. Relationships: is a type of somatic diversification of immune receptors via germline recombination within a single locus [GO:0002562]; is_a somatic diversification of immunoglobulins [GO:0016445] Sources: GOC:add, ISBN:0781735149 Also known as: somatic recombination of antibody gene segments Subtypes: somatic recombination of immunoglobulin genes involved in immune response [GO:0002204], B cell receptor editing [GO:0002452], immunoglobulin V(D)J recombination [GO:0033152]